{
  "gene": "UniProtKB:P0C7Q5",
  "term_id": "UNKNOWN:0001",
  "term_label": "Unknown molecular function",
  "gene_name": "Putative solute carrier family 35 member G4",
  "gene_symbol": "SLC35G4"
}